{
  "term_label": "Unknown biological process",
  "term_id": "UNKNOWN:0002",
  "gene_name": "Uncharacterized protein C12orf71",
  "gene": "UniProtKB:A8MTZ7",
  "gene_symbol": "C12orf71"
}